{
  "term_label": "regulation of transcription by RNA polymerase II",
  "gene_name": "Zinc finger protein 69 homolog",
  "gene_symbol": "ZFP69",
  "term_id": "GO:0006357",
  "gene": "UniProtKB:Q49AA0"
}